(-)-menthol dehydrogenase activity [GO:0047504] (MF) Definition: Catalysis of the reaction: (-)-menthol + NADP+ = (2S,5R)-menthone + H+ + NADPH. Sources: EC:1.1.1.207, RHEA:13917 Also known as: monoterpenoid dehydrogenase activity, (-)-menthol:NADP+ oxidoreductase activity Relationships: is a type of oxidoreductase activity, acting on the CH-OH group of donors, NAD or NADP as acceptor [GO:0016616]